{
  "gene": "UniProtKB:Q6P9G9",
  "term_label": "Unknown cellular component",
  "term_id": "UNKNOWN:0003",
  "gene_name": "Zinc finger protein 449",
  "gene_symbol": "ZNF449"
}